{
  "term_label": "Unknown molecular function",
  "gene_symbol": "SPATA31A7",
  "gene": "UniProtKB:Q8IWB4",
  "term_id": "UNKNOWN:0001",
  "gene_name": "Spermatogenesis-associated protein 31A7"
}